{
  "term_id": "GO:0032040",
  "term_label": "small-subunit processome",
  "gene_name": "U3 small nucleolar ribonucleoprotein protein IMP3",
  "gene": "UniProtKB:Q9NV31",
  "gene_symbol": "IMP3"
}